{
  "gene_name": "Cadherin-related family member 1",
  "term_id": "GO:0007155",
  "gene": "UniProtKB:Q96JP9",
  "term_label": "cell adhesion",
  "gene_symbol": "CDHR1"
}